{
  "gene": "UniProtKB:P05106",
  "gene_name": "Integrin beta-3",
  "term_label": "platelet aggregation",
  "term_id": "GO:0070527",
  "gene_symbol": "ITGB3"
}